{
  "term_label": "regulation of cell shape",
  "term_id": "GO:0008360",
  "gene_symbol": "NF2",
  "gene": "UniProtKB:P35240",
  "gene_name": "Merlin"
}